{
  "term_id": "GO:0042605",
  "gene_name": "HLA class II histocompatibility antigen, DO alpha chain",
  "gene_symbol": "HLA-DOA",
  "gene": "UniProtKB:P06340",
  "term_label": "peptide antigen binding"
}